{
  "gene_name": "Perforin-1",
  "gene_symbol": "PRF1",
  "gene": "UniProtKB:P14222",
  "term_id": "GO:0001771",
  "term_label": "immunological synapse formation"
}